{
  "term_label": "NEDD8 transferase activity",
  "gene_symbol": "UBE2F",
  "gene": "UniProtKB:Q969M7",
  "term_id": "GO:0019788",
  "gene_name": "NEDD8-conjugating enzyme UBE2F"
}